{
  "gene_name": "Liprin-beta-2",
  "gene": "UniProtKB:Q8ND30",
  "term_label": "Unknown molecular function",
  "gene_symbol": "PPFIBP2",
  "term_id": "UNKNOWN:0001"
}